{
  "gene_symbol": "CABP4",
  "term_id": "GO:0005246",
  "gene_name": "Calcium-binding protein 4",
  "term_label": "calcium channel regulator activity",
  "gene": "UniProtKB:P57796"
}